{
  "gene_symbol": "EMX2",
  "gene_name": "Homeobox protein EMX2",
  "term_id": "GO:0007420",
  "term_label": "brain development",
  "gene": "UniProtKB:Q04743"
}